detection of reduced oxygen by chemoreceptor signaling [GO:0003020] (biological process) Relationships: is a type of detection of hypoxia [GO:0070483]; is part of detection of hypoxic conditions in blood by chemoreceptor signaling [GO:0002007] Sources: GOC:mtg_cardio, ISBN:0323031951 Also known as: detection of reduced oxygen by chemoreceptor signalling Subtypes: detection of reduced oxygen by aortic body chemoreceptor signaling [GO:0003038], detection of reduced oxygen by carotid body chemoreceptor signaling [GO:0003039] Definition: The process in which information about the levels of oxygen are received and are converted to a molecular signal by chemoreceptors in the carotid bodies and the aortic bodies.